{
  "gene_symbol": "CMC2",
  "gene_name": "COX assembly mitochondrial protein 2 homolog",
  "term_id": "GO:0005739",
  "term_label": "mitochondrion",
  "gene": "UniProtKB:Q9NRP2"
}